{
  "gene_symbol": "AP1M1",
  "term_id": "GO:0030121",
  "gene": "UniProtKB:Q9BXS5",
  "term_label": "AP-1 adaptor complex",
  "gene_name": "AP-1 complex subunit mu-1"
}